{
  "gene": "UniProtKB:Q9NSD9",
  "term_label": "Unknown molecular function",
  "term_id": "UNKNOWN:0001",
  "gene_name": "Phenylalanine--tRNA ligase beta subunit",
  "gene_symbol": "FARSB"
}